histone H4K12 deacetylase activity, hydrolytic mechanism [GO:0140937] (molecular function) Definition: Catalysis of the reaction: histone H4 N6-acetyl-L-lysine (position 12) + H2O = histone H4 L-lysine (position 12) + acetate. This reaction represents the removal of an acetyl group from lysine at position 12 of the histone H4 protein. Note: Note that the residue position corresponds to the canonical human H4 histone (UniProtKB:P02309); this residue is conserved across all eukaryotes. Note that the initiation methionine is cleaved, so the first residue is S1. Also known as: histone H4K12 deacetylase activity, histone H4-K12 deacetylase activity, histone deacetylase activity (H4-K12 specific), histone H4-K12 deacetylation, histone H4K12 deacetylation Relationships: is a type of histone H4K deacetylase activity [GO:0141051]; is a type of histone deacetylase activity, hydrolytic mechanism [GO:0141221] References: PMID:15293224 Sources: GOC:vw